{
  "gene_symbol": "NKX6-2",
  "gene_name": "Homeobox protein Nkx-6.2",
  "term_id": "GO:0030154",
  "term_label": "cell differentiation",
  "gene": "UniProtKB:Q9C056"
}